regulation of thymocyte migration [GO:2000410] (biological process) Definition: Any process that modulates the frequency, rate or extent of thymocyte migration. Sources: GOC:mah Relationships: is a type of regulation of T cell migration [GO:2000404]; regulates thymocyte migration [GO:0072679] Also known as: regulation of thymic lymphocyte migration, regulation of immature T cell migration, regulation of immature T lymphocyte migration, regulation of immature T-cell migration, regulation of immature T-lymphocyte migration Subtypes: negative regulation of thymocyte migration [GO:2000411], positive regulation of thymocyte migration [GO:2000412], GO:2000413